interleukin-17-mediated signaling pathway [GO:0097400] (biological process) Definition: The series of molecular signals initiated by interleukin-17 binding to its receptor on the surface of a target cell, and ending with the regulation of a downstream cellular process, e.g. transcription. References: PMID:21602493 Sources: GOC:ic Also known as: IL-17-mediated signaling pathway, IL-17-mediated signalling pathway, interleukin-17-mediated signalling pathway Relationships: is a type of cytokine-mediated signaling pathway [GO:0019221]; is part of cellular response to interleukin-17 [GO:0097398] Regulation: regulated by GO:1903881; negatively regulated by GO:1903882; positively regulated by positive regulation of interleukin-17-mediated signaling pathway [GO:1903883]